protein K63-linked deubiquitination [GO:0070536] (biological process) References: PMID:19202061, PMID:19214193 Sources: GOC:mah Relationships: is a type of GO:0016579 Definition: A protein deubiquitination process in which a K63-linked ubiquitin chain, i.e. a polymer of ubiquitin formed by linkages between lysine residues at position 63 of the ubiquitin monomers, is removed from a protein. Regulation: regulated by regulation of protein K63-linked deubiquitination [GO:1903004]; negatively regulated by GO:1903005; positively regulated by positive regulation of protein K63-linked deubiquitination [GO:1903006]